{
  "term_label": "plasma membrane",
  "gene_name": "Melanocortin receptor 4",
  "gene": "UniProtKB:P32245",
  "term_id": "GO:0005886",
  "gene_symbol": "MC4R"
}